{
  "gene_name": "Ubiquitin carboxyl-terminal hydrolase 17-like protein 6",
  "term_label": "cytosol",
  "term_id": "GO:0005829",
  "gene": "UniProtKB:Q6QN14",
  "gene_symbol": "USP17L6P"
}